UDP-N-acetylmuramate dehydrogenase activity [GO:0008762] (molecular function) Also known as: MurB reductase, UDP-GlcNAc-enoylpyruvate reductase activity, UDP-N-acetylenolpyruvoylglucosamine reductase activity, UDP-N-acetylglucosamine-enoylpyruvate reductase activity, UDP-N-acetylmuramate:NADP+ oxidoreductase activity, uridine diphospho-N-acetylglucosamine-enolpyruvate reductase activity, uridine diphosphoacetylpyruvoylglucosamine reductase activity, uridine-5'-diphospho-N-acetyl-2-amino-2-deoxy-3-O-lactylglucose:NADP-oxidoreductase activity Definition: Catalysis of the reaction: UDP-N-acetylmuramate + NADP+ = UDP-N-acetyl-3-O-(1-carboxyvinyl)-D-glucosamine + NADPH + H+. Relationships: is a type of GO:0016616 Sources: EC:1.3.1.98